S100A9 complex [GO:1990662] (cellular component) Definition: A protein complex composed of a S100A9 dimer and capable of binding to toll-like receptor 4 (TLR4) and the receptor for advanced glycation end products (RAGE) initiating signal transduction through NF-kappa-B pathways. Transports arachidonic acid between the cytosol and the NADPH oxidase complex at the plasma membrane in neutrophils as part of an inflammatory signal cascade leading to an oxidative burst. Complexes with microtubules to increase cell motility. References: PMID:15642721 Sources: GOC:bhm Also known as: S100A9 homodimer Note: An example of this is S100A9 in human (UniProt symbol P06702) in PMID:15642721 (inferred from direct assay). Relationships: is a type of transmembrane transporter complex [GO:1902495]